{
  "gene_name": "N-acetylmuramoyl-L-alanine amidase",
  "term_id": "GO:0016019",
  "term_label": "peptidoglycan immune receptor activity",
  "gene_symbol": "PGLYRP2",
  "gene": "UniProtKB:Q96PD5"
}